{
  "term_label": "phagocytic cup",
  "gene_symbol": "BIN2",
  "gene": "UniProtKB:Q9UBW5",
  "term_id": "GO:0001891",
  "gene_name": "Bridging integrator 2"
}